regulation of modification of postsynaptic structure [GO:0099159] (biological process) Sources: GOC:dos Subtypes: GO:1905274 Relationships: is a type of regulation of modification of synaptic structure [GO:1905244]; RO_0002211 modification of postsynaptic structure [GO:0099010] Definition: Any process that modulates the frequency, rate or extent of modification of postsynaptic structure. Also known as: regulation of postsynapse remodelling